{
  "gene_symbol": "MRNIP",
  "gene": "UniProtKB:Q6NTE8",
  "term_id": "GO:0003682",
  "gene_name": "MRN complex-interacting protein",
  "term_label": "chromatin binding"
}